{
  "gene_symbol": "ZIC4",
  "gene": "UniProtKB:Q8N9L1",
  "gene_name": "Zinc finger protein ZIC 4",
  "term_id": "GO:0005634",
  "term_label": "nucleus"
}